{
  "gene_name": "Leukocyte receptor cluster member 9",
  "gene": "UniProtKB:Q96B70",
  "gene_symbol": "LENG9",
  "term_label": "Unknown biological process",
  "term_id": "UNKNOWN:0002"
}